{
  "gene_name": "Cytoskeleton-associated protein 5",
  "gene_symbol": "CKAP5",
  "gene": "UniProtKB:Q14008",
  "term_id": "GO:0061863",
  "term_label": "microtubule plus end polymerase"
}